unsaturated rhamnogalacturonyl hydrolase activity [GO:0102211] (molecular function) Relationships: is a type of hydrolase activity, hydrolyzing O-glycosyl compounds [GO:0004553] Sources: EC:3.2.1.172, GOC:pz Definition: Catalysis of the reaction: 2-O-(4-deoxy-beta-L-threo-hex-4-enopyranuronosyl)-alpha-L-rhamnopyranose(1-) + H2O = (4S,5S)-4,5-dihydroxy-2,6-dioxohexanoate + alpha-L-rhamnopyranose.